{
  "gene": "UniProtKB:P02743",
  "gene_symbol": "APCS",
  "term_label": "extracellular space",
  "gene_name": "Serum amyloid P-component",
  "term_id": "GO:0005615"
}